post-anaphase array microtubule end [GO:1905760] (cellular component) Relationships: is a type of microtubule end [GO:1990752]; is part of post-anaphase array microtubule [GO:1905759] Also known as: microtubule end of microtubule of PAA, microtubule end of microtubule of post-anaphase array, microtubule end of microtubule of post-anaphase microtubule array, microtubule end of microtubuli of PAA, microtubule end of microtubuli of post-anaphase array, microtubule end of microtubuli of post-anaphase microtubule array, microtubule end of microtubulus of PAA, microtubule end of microtubulus of post-anaphase array, microtubule end of microtubulus of post-anaphase microtubule array, microtubule end of post-anaphase array microtubule, microtubule end of neurotubule of PAA, microtubule end of neurotubule of post-anaphase array, microtubule end of neurotubule of post-anaphase microtubule array Definition: Any microtubule end that is part of a post-anaphase array microtubule. References: PMID:11007487 Sources: GOC:TermGenie, GO_REF:0000064